histone H2B C-terminal K residue ubiquitin ligase activity [GO:0140850] (molecular function) References: PMID:17363370, PMID:28624371 Definition: Catalysis of the transfer of a ubiquitin molecule to a histone 2B at the conserved C-terminal lysine (K) residue. The last K residue is at position 119 in fission yeast, 123 in budding yeast, and 120 in mammals. Also known as: histone H2B conserved C-terminal lysine ubiquitin ligase activity, histone H2B-K120 ubiquitin ligase activity, histone H2BK120 ubiquitin ligase activity, histone ubiquitin ligase activity (H2B-K120 specific) Relationships: is a type of GO:0141054